{
  "gene": "UniProtKB:Q9ULH4",
  "term_id": "UNKNOWN:0001",
  "gene_name": "Leucine-rich repeat and fibronectin type-III domain-containing protein 2",
  "gene_symbol": "LRFN2",
  "term_label": "Unknown molecular function"
}